{
  "term_label": "kidney development",
  "gene": "UniProtKB:Q9NPC8",
  "gene_symbol": "SIX2",
  "gene_name": "Homeobox protein SIX2",
  "term_id": "GO:0001822"
}